{
  "term_id": "UNKNOWN:0002",
  "gene_name": "Heparin cofactor 2",
  "gene": "UniProtKB:P05546",
  "gene_symbol": "SERPIND1",
  "term_label": "Unknown biological process"
}